{
  "term_label": "protein serine/threonine kinase activity",
  "gene_name": "Serine_threonine-protein kinase PLK2",
  "gene_symbol": "PLK2",
  "gene": "UniProtKB:Q9NYY3",
  "term_id": "GO:0004674"
}